{
  "term_id": "GO:0043484",
  "term_label": "regulation of RNA splicing",
  "gene_name": "Polypyrimidine tract-binding protein 1",
  "gene": "UniProtKB:P26599",
  "gene_symbol": "PTBP1"
}